{
  "term_label": "lens development in camera-type eye",
  "gene_name": "Beta-crystallin A3",
  "gene_symbol": "CRYBA1",
  "gene": "UniProtKB:P05813",
  "term_id": "GO:0002088"
}